{
  "gene_symbol": "KIF19",
  "term_id": "GO:0008017",
  "gene_name": "Kinesin-like protein KIF19",
  "term_label": "microtubule binding",
  "gene": "UniProtKB:Q2TAC6"
}